daphnetin-8-O-methyltransferase activity [GO:0102358] (molecular function) Sources: RHEA:68960 Relationships: is a type of methyltransferase activity [GO:0008168] Definition: Catalysis of the reaction: 7,8-dihydroxycoumarin + S-adenosyl-L-methionine = 7-hydroxy-8-methoxycoumarin + H+ + S-adenosyl-L-homocysteine.